{
  "gene_name": "Uncharacterized protein C2orf81",
  "gene": "UniProtKB:A6NN90",
  "term_id": "UNKNOWN:0001",
  "term_label": "Unknown molecular function",
  "gene_symbol": "C2orf81"
}